positive regulation of dopamine receptor signaling pathway [GO:0060161] (biological process) Definition: Any process that activates or increases the frequency, rate or extent of the dopamine receptor protein signaling pathway. A dopamine receptor signaling pathway is the series of molecular signals generated as a consequence of a dopamine receptor binding to one of its physiological ligands. Sources: GOC:dph Also known as: positive regulation of dopamine receptor signalling pathway Relationships: is a type of positive regulation of G protein-coupled receptor signaling pathway [GO:0045745]; is_a regulation of dopamine receptor signaling pathway [GO:0060159]; positively regulates G protein-coupled dopamine receptor signaling pathway [GO:0007212] Subtypes: positive regulation of adenylate cyclase-inhibiting dopamine receptor signaling pathway [GO:1904992]